SMAD protein signal transduction [GO:0060395] (biological process) Definition: An intracellular signaling cassette that starts with the activation of a SMAD protein, leading to the formation of a complex with co-SMADs, which translocates to the nucleus and regulates transcription of specific target genes. Sources: GOC:BHF Relationships: is a type of GO:0141124; is part of cell surface receptor protein serine/threonine kinase signaling pathway [GO:0007178] Regulation: RO_0002211 by regulation of SMAD protein signal transduction [GO:0060390]; positively regulated by positive regulation of SMAD protein signal transduction [GO:0060391]; negatively regulated by negative regulation of SMAD protein signal transduction [GO:0060392] Note: Note that the upstream receptor and its ligand regulate the pathway (and are not part of the SMAD pathway), since it is an intracellular signaling pathway.